{
  "gene_symbol": "PPP1R13L",
  "gene_name": "RelA-associated inhibitor",
  "term_label": "Unknown molecular function",
  "gene": "UniProtKB:Q8WUF5",
  "term_id": "UNKNOWN:0001"
}